{
  "gene": "UniProtKB:P0CG08",
  "term_label": "intracellular pH reduction",
  "term_id": "GO:0051452",
  "gene_symbol": "GPR89B",
  "gene_name": "Golgi pH regulator B"
}